extracellular regulation of signal transduction [GO:1900115] (biological process) Also known as: regulation of signaling pathway in extracellular region, regulation of signalling pathway in extracellular region Definition: Any regulation of signal transduction that takes place in the extracellular region. Subtypes: extracellular negative regulation of signal transduction [GO:1900116] Relationships: is a type of regulation of signal transduction [GO:0009966]; occurs in extracellular region [GO:0005576] Sources: GOC:TermGenie, GOC:signaling